long-chain fatty aldehyde oxidative decarbonylase activity [GO:0160238] (molecular function) Also known as: aldehyde oxidative decarbonylase activity References: PMID:22927409 Sources: RHEA:83563 Relationships: is a type of carbon-carbon lyase activity [GO:0016830] Definition: Catalysis of the reaction: reduced [NADPH-hemoprotein reductase] + O2 + a long-chain fatty aldehyde = oxidized [NADPH-hemoprotein reductase] + CO2 + H2O + H+ + a long-chain alkane.